{
  "gene_name": "Uncharacterized protein C14orf93",
  "gene": "UniProtKB:Q9H972",
  "term_id": "UNKNOWN:0003",
  "gene_symbol": "C14orf93",
  "term_label": "Unknown cellular component"
}